early neuron differentiation in forebrain [GO:0021862] (biological process) Relationships: is a type of forebrain neuron differentiation [GO:0021879] References: PMID:16226447 Sources: GOC:cls, GOC:dgh, GOC:dph, GOC:jid, GO_REF:0000021 Definition: The process in which neuroepithelial cells in the neural tube acquire specialized structural and/or functional features of neurons. Differentiation includes the processes involved in commitment of a cell to a specific fate.